{
  "gene_symbol": "TMEM184C",
  "gene": "UniProtKB:Q9NVA4",
  "term_id": "GO:0016020",
  "gene_name": "Transmembrane protein 184C",
  "term_label": "membrane"
}